lipoprotein modification [GO:0042160] (biological process) Relationships: is a type of lipoprotein metabolic process [GO:0042157] Subtypes: lipoprotein oxidation [GO:0042161] Sources: GOC:mah Definition: The chemical reactions and pathways resulting in the covalent alteration of one or more amino acid or lipid residues occurring in a lipoprotein, any conjugated, water-soluble protein in which the nonprotein group consists of a lipid or lipids.